{
  "gene": "UniProtKB:Q9BY89",
  "gene_name": "Uncharacterized protein KIAA1671",
  "gene_symbol": "KIAA1671",
  "term_id": "UNKNOWN:0002",
  "term_label": "Unknown biological process"
}